5-(carboxyamino)imidazole ribonucleotide synthase activity [GO:0034028] (molecular function) Definition: Catalysis of the reaction: 5-amino-1-(5-phospho-D-ribosyl)imidazole + ATP + bicarbonate = 5-carboxyamino-1-(5-phospho-D-ribosyl)imidazole + ADP + 3 H+ + phosphate. Sources: EC:6.3.4.18, RHEA:19317 Relationships: is a type of GO:0016879 Also known as: 5-amino-1-(5-phospho-D-ribosyl)imidazole:carbon-dioxide ligase (ADP-forming) activity, N5-CAIR synthetase activity, N5-carboxyaminoimidazole ribonucleotide synthetase activity, PurK